pyrimidine nucleotide transmembrane transporter activity [GO:0015218] (molecular function) Sources: GOC:ai Definition: Enables the transfer of a pyrimidine nucleotide, any compound consisting of a pyrimidine nucleoside esterified with (ortho)phosphate, from one side of a membrane to the other. Relationships: is a type of nucleotide transmembrane transporter activity [GO:0015215]; is part of pyrimidine nucleotide transport [GO:0006864]